{
  "term_id": "GO:0004348",
  "term_label": "glucosylceramidase activity",
  "gene_name": "Lysosomal acid glucosylceramidase",
  "gene_symbol": "GBA1",
  "gene": "UniProtKB:P04062"
}